SUMO ligase complex [GO:0106068] (cellular component) Also known as: SUMO transferase complex, SUMO-protein ligase complex, Sumoylation complex Subtypes: GO:0030915, synapsis initiation complex [GO:0106069], activated SUMO-E1 ligase complex [GO:1990354] Relationships: is a type of GO:1990234 Definition: A protein ligase complex that enables protein sumoylation. Consists of a SUMO-protein transferase and other proteins that may confer substrate specificity of the complex. References: PMID:16847351